{
  "gene": "UniProtKB:Q96JM4",
  "gene_symbol": "LRRIQ1",
  "gene_name": "Leucine-rich repeat and IQ domain-containing protein 1",
  "term_id": "UNKNOWN:0001",
  "term_label": "Unknown molecular function"
}